thalamus development [GO:0021794] (biological process) Definition: The process in which the thalamus changes over time, from its initial formation to its mature state. Sources: GOC:cls, GOC:dgh, GOC:dph, GOC:jid, GO_REF:0000021 Relationships: is a type of GO:0048856; is part of diencephalon development [GO:0021536]